{
  "gene_symbol": "EPHX2",
  "term_id": "GO:0042577",
  "gene": "UniProtKB:P34913",
  "gene_name": "Bifunctional epoxide hydrolase 2",
  "term_label": "lipid phosphatase activity"
}